{
  "term_label": "vacuolar membrane",
  "gene_name": "ATP-binding cassette sub-family B member 6",
  "gene_symbol": "ABCB6",
  "gene": "UniProtKB:Q9NP58",
  "term_id": "GO:0005774"
}